protein localization to nucleolus [GO:1902570] (biological process) Definition: A process in which a protein is transported to, or maintained in, a location within a nucleolus. References: PMID:22809626 Sources: GOC:TermGenie Also known as: protein localisation in nucleolus, protein localisation to nucleolus, protein localization in nucleolus Relationships: is a type of GO:0034504 Regulation: regulated by regulation of protein localization to nucleolus [GO:1904749]; RO_0002212 by negative regulation of protein localization to nucleolus [GO:1904750]; positively regulated by positive regulation of protein localization to nucleolus [GO:1904751]